{
  "gene": "UniProtKB:O60543",
  "gene_name": "Lipid transferase CIDEA",
  "term_label": "lipid storage",
  "gene_symbol": "CIDEA",
  "term_id": "GO:0019915"
}